dendritic knob [GO:0098788] (cellular component) Relationships: is a type of dendrite terminus [GO:0044292] Also known as: apical dendritic knob Definition: The terminal swelling of an apical dendrite of a ciliated olfactory receptor neuron. Each knob gives rise to 5 to 20 long delicate nonmotile cilia, which extend into the mucus covering the sensory epithelium. References: PMID:20801626